{
  "gene_symbol": "PTPN1",
  "gene": "UniProtKB:P18031",
  "term_label": "non-membrane spanning protein tyrosine phosphatase activity",
  "gene_name": "Tyrosine-protein phosphatase non-receptor type 1",
  "term_id": "GO:0004726"
}